{
  "term_label": "arylsulfatase activity",
  "gene_symbol": "ARSL",
  "gene": "UniProtKB:P51690",
  "term_id": "GO:0004065",
  "gene_name": "Arylsulfatase L"
}